{
  "gene_symbol": "ASB9",
  "term_id": "GO:0016567",
  "gene_name": "Ankyrin repeat and SOCS box protein 9",
  "term_label": "protein ubiquitination",
  "gene": "UniProtKB:Q96DX5"
}